DNA-templated DNA replication [GO:0006261] (biological process) Subtypes: GO:0001326, GO:0006264, plastid DNA replication [GO:0033259], cell cycle DNA replication [GO:0044786], rolling circle DNA replication [GO:0070581], theta DNA replication [GO:0070582] Definition: A DNA replication process that uses parental DNA as a template for the DNA-dependent DNA polymerases that synthesize the new strands. Sources: GOC:mah, ISBN:0198506732 Relationships: is a type of GO:0006260 Also known as: DNA-dependent DNA replication Regulation: regulated by regulation of DNA-templated DNA replication [GO:0090329]; negatively regulated by negative regulation of DNA-templated DNA replication [GO:2000104]; positively regulated by GO:2000105